{
  "gene_symbol": "TMCO2",
  "term_label": "Unknown cellular component",
  "gene": "UniProtKB:Q7Z6W1",
  "gene_name": "Transmembrane and coiled-coil domain-containing protein 2",
  "term_id": "UNKNOWN:0003"
}